{
  "term_id": "GO:0000981",
  "gene": "UniProtKB:Q96NK8",
  "gene_name": "Neurogenic differentiation factor 6",
  "gene_symbol": "NEUROD6",
  "term_label": "DNA-binding transcription factor activity, RNA polymerase II-specific"
}